{
  "term_id": "UNKNOWN:0002",
  "gene_name": "NADH dehydrogenase [ubiquinone] 1 alpha subcomplex subunit 13",
  "gene_symbol": "NDUFA13",
  "gene": "UniProtKB:Q9P0J0",
  "term_label": "Unknown biological process"
}